{
  "gene_name": "Twinfilin-2",
  "gene": "UniProtKB:Q6IBS0",
  "term_id": "GO:0030042",
  "gene_symbol": "TWF2",
  "term_label": "actin filament depolymerization"
}